{
  "term_id": "GO:0005634",
  "gene_name": "Pre-mRNA-processing factor 39",
  "term_label": "nucleus",
  "gene_symbol": "PRPF39",
  "gene": "UniProtKB:Q86UA1"
}